NF-kappaB complex [GO:0071159] (CC) Sources: ISBN:0849327946 Subtypes: GO:0035525 Definition: A protein complex that consists of a homo- or heterodimer of members of a family of structurally related proteins that contain a conserved N-terminal region called the Rel homology domain (RHD). In the nucleus, NF-kappaB complexes act as transcription factors. In unstimulated cells, NF-kappaB dimers are sequestered in the cytoplasm by IkappaB monomers; signals that induce NF-kappaB activity cause degradation of IkappaB, allowing NF-kappaB dimers to translocate to the nucleus and induce gene expression. Relationships: is a type of nuclear protein-containing complex [GO:0140513]